{
  "term_label": "Unknown cellular component",
  "gene_name": "Elongin-A2",
  "gene_symbol": "ELOA2",
  "gene": "UniProtKB:Q8IYF1",
  "term_id": "UNKNOWN:0003"
}